{
  "gene_symbol": "AAGAB",
  "term_id": "UNKNOWN:0002",
  "gene_name": "Alpha- and gamma-adaptin-binding protein p34",
  "term_label": "Unknown biological process",
  "gene": "UniProtKB:Q6PD74"
}